{
  "term_id": "UNKNOWN:0002",
  "gene_name": "Lengsin",
  "gene": "UniProtKB:Q5TDP6",
  "gene_symbol": "LGSN",
  "term_label": "Unknown biological process"
}